proximal/distal axis specification [GO:0009946] (biological process) Definition: The establishment, maintenance and elaboration of the proximal/distal axis. The proximal/distal axis is defined by a line that runs from main body (proximal end) of an organism outward (distal end). Sources: GOC:dph, GOC:go_curators, GOC:tb Also known as: proximodistal axis specification, proximal/distal axis determination Relationships: is a type of axis specification [GO:0009798]; BFO_0000050 GO:0009954 Subtypes: GO:0061115